{
  "gene_symbol": "MAP4K3",
  "term_label": "intracellular signal transduction",
  "gene": "UniProtKB:Q8IVH8",
  "gene_name": "Mitogen-activated protein kinase kinase kinase kinase 3",
  "term_id": "GO:0035556"
}